{
  "term_label": "regulation of synaptic transmission, glutamatergic",
  "gene": "UniProtKB:Q9NSC5",
  "term_id": "GO:0051966",
  "gene_symbol": "HOMER3",
  "gene_name": "Homer protein homolog 3"
}